{
  "gene": "UniProtKB:Q8TAM6",
  "gene_symbol": "ERMN",
  "term_label": "filopodium",
  "term_id": "GO:0030175",
  "gene_name": "Ermin"
}